{
  "gene": "UniProtKB:Q86W24",
  "gene_name": "NACHT, LRR and PYD domains-containing protein 14",
  "term_label": "cytoplasm",
  "term_id": "GO:0005737",
  "gene_symbol": "NLRP14"
}